{
  "gene": "UniProtKB:O00167",
  "gene_symbol": "EYA2",
  "gene_name": "Eyes absent homolog 2",
  "term_id": "GO:0004725",
  "term_label": "protein tyrosine phosphatase activity"
}